{
  "gene_name": "Nitric oxide synthase, inducible",
  "term_label": "defense response to bacterium",
  "term_id": "GO:0042742",
  "gene": "UniProtKB:P35228",
  "gene_symbol": "NOS2"
}